{
  "gene_symbol": "ANXA8L1",
  "term_id": "GO:0005544",
  "gene_name": "Annexin A8-like protein 1",
  "term_label": "calcium-dependent phospholipid binding",
  "gene": "UniProtKB:Q5VT79"
}